{
  "term_id": "GO:0072657",
  "term_label": "protein localization to membrane",
  "gene": "UniProtKB:O15321",
  "gene_symbol": "TM9SF1",
  "gene_name": "Transmembrane 9 superfamily member 1"
}